{
  "gene_name": "Olfactory receptor 2C1",
  "gene_symbol": "OR2C1",
  "term_label": "detection of chemical stimulus involved in sensory perception of smell",
  "gene": "UniProtKB:O95371",
  "term_id": "GO:0050911"
}